{
  "gene_name": "Necdin",
  "gene_symbol": "NDN",
  "gene": "UniProtKB:Q99608",
  "term_id": "GO:0005634",
  "term_label": "nucleus"
}